{
  "term_id": "GO:0042564",
  "gene_symbol": "KPNA7",
  "gene_name": "Importin subunit alpha-8",
  "gene": "UniProtKB:A9QM74",
  "term_label": "NLS-dependent protein nuclear import complex"
}